{
  "term_label": "cytoplasm",
  "gene_symbol": "CAPN2",
  "gene_name": "Calpain-2 catalytic subunit",
  "gene": "UniProtKB:P17655",
  "term_id": "GO:0005737"
}